{
  "gene": "UniProtKB:P53597",
  "term_label": "mitochondrion",
  "term_id": "GO:0005739",
  "gene_symbol": "SUCLG1",
  "gene_name": "Succinate--CoA ligase [ADP_GDP-forming] subunit alpha, mitochondrial"
}